centromeric sister chromatid cohesion [GO:0070601] (biological process) Definition: The cell cycle process in which the sister chromatids of a replicated chromosome are joined along the length of the centromeric region of the chromosome. Sources: GOC:mah Also known as: sister chromatid cohesion at centromere Relationships: is a type of sister chromatid cohesion [GO:0007062] Subtypes: meiotic sister chromatid cohesion, centromeric [GO:0051754], mitotic sister chromatid cohesion, centromeric [GO:0071962] Regulation: RO_0002211 by regulation of centromeric sister chromatid cohesion [GO:0070602]